{
  "gene_symbol": "AP4S1",
  "term_label": "Unknown molecular function",
  "gene_name": "AP-4 complex subunit sigma-1",
  "gene": "UniProtKB:Q9Y587",
  "term_id": "UNKNOWN:0001"
}